{
  "term_label": "extracellular space",
  "gene_symbol": "WNT11",
  "gene": "UniProtKB:O96014",
  "term_id": "GO:0005615",
  "gene_name": "Protein Wnt-11"
}